{
  "term_label": "mitotic cytokinetic process",
  "gene": "UniProtKB:Q8IXV7",
  "gene_name": "Kelch domain-containing protein 8B",
  "gene_symbol": "KLHDC8B",
  "term_id": "GO:1902410"
}